{
  "gene_name": "ORM1-like protein 3",
  "gene_symbol": "ORMDL3",
  "gene": "UniProtKB:Q8N138",
  "term_label": "serine palmitoyltransferase complex",
  "term_id": "GO:0017059"
}